{
  "gene": "UniProtKB:Q9UHE8",
  "term_label": "Unknown biological process",
  "term_id": "UNKNOWN:0002",
  "gene_symbol": "STEAP1",
  "gene_name": "Metalloreductase STEAP1"
}